{
  "term_id": "UNKNOWN:0002",
  "term_label": "Unknown biological process",
  "gene_symbol": "BVES-AS1",
  "gene": "UniProtKB:Q5T3Y7",
  "gene_name": "Putative uncharacterized protein BVES-AS1"
}